{
  "gene": "UniProtKB:Q96FT9",
  "gene_symbol": "IFT43",
  "term_label": "Unknown molecular function",
  "gene_name": "Intraflagellar transport protein 43 homolog",
  "term_id": "UNKNOWN:0001"
}